{
  "gene": "UniProtKB:Q5T1S8",
  "term_label": "Schmidt-Lanterman incisure",
  "gene_name": "Noncompact myelin-associated protein",
  "gene_symbol": "NCMAP",
  "term_id": "GO:0043220"
}